{
  "gene_name": "Protein phosphatase 1D",
  "gene": "UniProtKB:O15297",
  "term_id": "GO:0004722",
  "term_label": "protein serine/threonine phosphatase activity",
  "gene_symbol": "PPM1D"
}